extension of a leading process involved in cell motility in cerebral cortex radial glia guided migration [GO:0021816] (biological process) Definition: The rearrangements of the microtubule cytoskeleton that result in the extension of a leading process, where this process is involved in the movement of cells along radial glial cells. References: PMID:12626695 Sources: GOC:cls, GOC:dgh, GOC:dph, GOC:jid, GO_REF:0000021 Relationships: is_a modulation of microtubule cytoskeleton involved in cerebral cortex radial glia guided migration [GO:0021815]; is a type of pseudopodium assembly [GO:0031269]